4-nitrobenzyl alcohol oxidase activity [GO:0102038] (molecular function) Sources: GOC:pz Definition: Catalysis of the reaction: 4-nitrobenzyl alcohol + O2 = 4-nitrobenzaldehyde + hydrogen peroxide. Relationships: is a type of oxidoreductase activity, acting on the CH-OH group of donors, oxygen as acceptor [GO:0016899]